{
  "gene_symbol": "BLK",
  "term_id": "GO:0004715",
  "term_label": "non-membrane spanning protein tyrosine kinase activity",
  "gene": "UniProtKB:P51451",
  "gene_name": "Tyrosine-protein kinase Blk"
}